photosynthetic acclimation [GO:0009643] (biological process) Also known as: light acclimatization, photoacclimation Definition: A response to light intensity in which exposure to medium-intensity light results in increased tolerance to high-intensity light. References: PMID:11069694 Sources: GOC:mah Relationships: is a type of response to light intensity [GO:0009642]